L-tyrosine catabolic process to fumarate [GO:0019445] (biological process) Also known as: tyrosine breakdown to fumarate, tyrosine degradation to fumarate Relationships: is a type of fumarate metabolic process [GO:0006106]; is a type of L-tyrosine catabolic process [GO:0006572]; is a type of dicarboxylic acid biosynthetic process [GO:0043650] Sources: GOC:go_curators Definition: The chemical reactions and pathways resulting in the breakdown of L-tyrosine into other compounds, including fumarate.